positive regulation of telomeric loop disassembly [GO:1904535] (biological process) Subtypes: positive regulation of telomeric D-loop disassembly [GO:1905840] References: PMID:22579284 Sources: GOC:BHF, GOC:BHF_telomere, GOC:TermGenie, GOC:nc, GO_REF:0000058 Definition: Any process that activates or increases the frequency, rate or extent of telomeric loop disassembly. Relationships: is a type of positive regulation of telomere maintenance [GO:0032206]; is a type of GO:1904533; positively regulates telomeric loop disassembly [GO:0090657] Also known as: positive regulation of T loop disassembly, up regulation of T loop disassembly, up regulation of telomeric loop disassembly, up-regulation of T loop disassembly, up-regulation of telomeric loop disassembly, upregulation of T loop disassembly, upregulation of telomeric loop disassembly, activation of T loop disassembly, activation of telomeric loop disassembly